{
  "gene_name": "ETS translocation variant 4",
  "gene_symbol": "ETV4",
  "gene": "UniProtKB:P43268",
  "term_label": "regulation of transcription by RNA polymerase II",
  "term_id": "GO:0006357"
}